neural crest cell fate commitment [GO:0014034] (biological process) Definition: The process in which a cell becomes committed to become a neural crest cell. Relationships: is a type of GO:0048865; is part of neural crest formation [GO:0014029]; is part of neural crest cell differentiation [GO:0014033] Sources: GOC:dh, GOC:ef